lung ciliated cell differentiation [GO:0061141] (BP) Definition: The process in which a relatively unspecialized cell acquires specialized features of a lung ciliated cell. A lung ciliated cell is a specialized lung epithelial cell that contains cilia for moving substances released from lung secretory cells. Relationships: is a type of lung epithelial cell differentiation [GO:0060487]; is a type of multi-ciliated epithelial cell differentiation [GO:1903251] Sources: GOC:cilia, GOC:dph, GOC:krc Regulation: regulated by GO:1901246; negatively regulated by negative regulation of lung ciliated cell differentiation [GO:1901247]; positively regulated by GO:1901248